{
  "term_id": "UNKNOWN:0002",
  "gene_name": "Inactive hydroxysteroid dehydrogenase-like protein 1",
  "term_label": "Unknown biological process",
  "gene_symbol": "HSDL1",
  "gene": "UniProtKB:Q3SXM5"
}